{
  "gene": "UniProtKB:P43119",
  "term_label": "positive regulation of cytosolic calcium ion concentration",
  "gene_symbol": "PTGIR",
  "gene_name": "Prostacyclin receptor",
  "term_id": "GO:0007204"
}